{
  "gene_name": "E3 ubiquitin-protein ligase ZFP91",
  "term_label": "Unknown molecular function",
  "gene_symbol": "ZFP91",
  "gene": "UniProtKB:Q96JP5",
  "term_id": "UNKNOWN:0001"
}